{
  "gene_symbol": "SLC25A20",
  "gene_name": "Mitochondrial carnitine_acylcarnitine carrier protein",
  "term_id": "GO:1902603",
  "gene": "UniProtKB:O43772",
  "term_label": "carnitine transmembrane transport"
}